{
  "gene": "UniProtKB:Q4VX62",
  "gene_symbol": "LINC02901",
  "term_label": "Unknown molecular function",
  "term_id": "UNKNOWN:0001",
  "gene_name": "Putative uncharacterized protein LINC02901"
}